{
  "term_label": "regulation of transcription by RNA polymerase II",
  "gene_name": "Bromodomain-containing protein 9",
  "term_id": "GO:0006357",
  "gene_symbol": "BRD9",
  "gene": "UniProtKB:Q9H8M2"
}